{
  "term_label": "regulatory ncRNA-mediated gene silencing",
  "term_id": "GO:0031047",
  "gene": "UniProtKB:Q7Z3Z3",
  "gene_symbol": "PIWIL3",
  "gene_name": "Piwi-like protein 3"
}